protein unfolding [GO:0043335] (biological process) Relationships: is a type of GO:0009987 Sources: GOC:mlg Definition: The process of assisting in the disassembly of non-covalent linkages in a protein or protein aggregate, often where the proteins are in a non-functional or denatured state.